{
  "gene_name": "DNA dC-dU-editing enzyme APOBEC-3C",
  "gene": "UniProtKB:Q9NRW3",
  "term_id": "GO:0005634",
  "gene_symbol": "APOBEC3C",
  "term_label": "nucleus"
}